glutathione peroxidase activity [GO:0004602] (molecular function) Relationships: is a type of peroxidase activity [GO:0004601] Definition: Catalysis of the reaction: 2 glutathione + hydrogen peroxide = oxidized glutathione + 2 H2O. References: PMID:36771108 Sources: EC:1.11.1.9 Also known as: non-selenium glutathione peroxidase activity, GSH peroxidase activity, glutathione:hydrogen-peroxide oxidoreductase activity, reduced glutathione peroxidase activity, selenium-glutathione peroxidase activity